{
  "gene": "UniProtKB:Q8NF50",
  "term_label": "cell leading edge",
  "gene_name": "Dedicator of cytokinesis protein 8",
  "term_id": "GO:0031252",
  "gene_symbol": "DOCK8"
}